{
  "term_id": "GO:0051642",
  "term_label": "centrosome localization",
  "gene_name": "Disks large-associated protein 5",
  "gene": "UniProtKB:Q15398",
  "gene_symbol": "DLGAP5"
}